{
  "term_id": "GO:0034271",
  "gene_symbol": "PIK3C3",
  "gene": "UniProtKB:Q8NEB9",
  "term_label": "phosphatidylinositol 3-kinase complex, class III, type I",
  "gene_name": "Phosphatidylinositol 3-kinase catalytic subunit type 3"
}